{
  "gene_name": "Alpha-crystallin A chain",
  "gene": "UniProtKB:P02489",
  "term_label": "lens development in camera-type eye",
  "term_id": "GO:0002088",
  "gene_symbol": "CRYAA"
}